{
  "term_id": "GO:0046513",
  "gene_name": "Ceramide synthase 3",
  "gene_symbol": "CERS3",
  "gene": "UniProtKB:Q8IU89",
  "term_label": "ceramide biosynthetic process"
}